sn-glycerol-3-phosphate 1-galactosyltransferase activity [GO:0047279] (molecular function) Relationships: is a type of UDP-galactosyltransferase activity [GO:0035250] Sources: EC:2.4.1.96, RHEA:20341 Also known as: UDP-Gal:sn-glycero-3-phosphoric acid 1-alpha-galactosyl-transferase activity, UDP-galactose:sn-glycerol-3-phosphate 1-alpha-D-galactosyltransferase activity, UDPgalactose:sn-glycerol-3-phosphate 1-alpha-D-galactosyltransferase activity, UDPgalactose:sn-glycerol-3-phosphate alpha-D-galactosyltransferase activity, glycerol 3-phosphate 1alpha-galactosyltransferase activity, isofloridoside-phosphate synthase activity, uridine diphosphogalactose-glycerol phosphate galactosyltransferase activity Definition: Catalysis of the reaction: sn-glycerol 3-phosphate + UDP-D-galactose = 1-O-alpha-D-galactosyl-sn-glycerol 3-phosphate + H+ + UDP.